asperfuranone catabolic process [GO:1900553] (BP) Also known as: asperfuranone breakdown, asperfuranone catabolism, asperfuranone degradation Relationships: is a type of polyketide catabolic process [GO:0030640]; is_a diol catabolic process [GO:0034313]; is a type of ketone catabolic process [GO:0042182]; is a type of tertiary alcohol metabolic process [GO:1902644]; is a type of secondary alcohol metabolic process [GO:1902652] Sources: GOC:TermGenie, GOC:di Definition: The chemical reactions and pathways resulting in the breakdown of asperfuranone.